{
  "gene_name": "T cell receptor beta variable 3-1",
  "gene_symbol": "TRBV3-1",
  "gene": "UniProtKB:A0A576",
  "term_label": "cell surface receptor signaling pathway",
  "term_id": "GO:0007166"
}